{
  "gene_symbol": "ADK",
  "gene_name": "Adenosine kinase",
  "term_label": "cytosol",
  "gene": "UniProtKB:P55263",
  "term_id": "GO:0005829"
}